regulation of ephrin receptor signaling pathway [GO:1901187] (biological process) Subtypes: negative regulation of ephrin receptor signaling pathway [GO:1901188], positive regulation of ephrin receptor signaling pathway [GO:1901189] Also known as: regulation of Eph receptor signaling pathway, regulation of Eph receptor signalling pathway Definition: Any process that modulates the frequency, rate or extent of ephrin receptor signaling pathway. Sources: GOC:BHF, GOC:TermGenie Relationships: is a type of regulation of signal transduction [GO:0009966]; regulates ephrin receptor signaling pathway [GO:0048013]